{
  "gene": "UniProtKB:Q6DRA6",
  "gene_symbol": "H2BC19P",
  "gene_name": "Putative histone H2B type 2-D",
  "term_id": "GO:0006325",
  "term_label": "chromatin organization"
}